acetyl-CoA transmembrane transporter activity [GO:0008521] (molecular function) Also known as: acetyl-CoA transporter activity Sources: GOC:ai Subtypes: acetyl-CoA:CoA antiporter activity [GO:0015325] Definition: Enables the transfer of acetyl-CoA from one side of a membrane to the other. Acetyl-CoA is a derivative of coenzyme A in which the sulfhydryl group is acetylated; it is a metabolite derived from several pathways (e.g. glycolysis, fatty acid oxidation, amino-acid catabolism) and is further metabolized by the tricarboxylic acid cycle. It is a key intermediate in lipid and terpenoid biosynthesis. Relationships: is a type of organophosphate ester transmembrane transporter activity [GO:0015605]; is_a nucleobase-containing compound transmembrane transporter activity [GO:0015932]; is a type of amide transmembrane transporter activity [GO:0042887]; is a type of sulfur compound transmembrane transporter activity [GO:1901682]; is part of GO:0015876